{
  "term_label": "Unknown molecular function",
  "gene": "UniProtKB:Q99437",
  "gene_name": "V-type proton ATPase 21 kDa proteolipid subunit c''",
  "term_id": "UNKNOWN:0001",
  "gene_symbol": "ATP6V0B"
}